{
  "gene_symbol": "SCFD1",
  "gene_name": "Sec1 family domain-containing protein 1",
  "term_id": "GO:0000139",
  "gene": "UniProtKB:Q8WVM8",
  "term_label": "Golgi membrane"
}